regulation of chloride transport [GO:2001225] (biological process) Definition: Any process that modulates the frequency, rate or extent of chloride transport. Sources: GOC:dph Relationships: is a type of regulation of monoatomic anion transport [GO:0044070]; regulates GO:0006821 Subtypes: negative regulation of chloride transport [GO:2001226]